{
  "gene_symbol": "FZD9",
  "term_label": "non-canonical Wnt signaling pathway",
  "term_id": "GO:0035567",
  "gene": "UniProtKB:O00144",
  "gene_name": "Frizzled-9"
}